{
  "term_id": "UNKNOWN:0001",
  "gene": "UniProtKB:Q5JXC2",
  "term_label": "Unknown molecular function",
  "gene_symbol": "MIIP",
  "gene_name": "Migration and invasion-inhibitory protein"
}